{
  "gene_symbol": "THYN1",
  "term_label": "nucleus",
  "gene": "UniProtKB:Q9P016",
  "term_id": "GO:0005634",
  "gene_name": "Thymocyte nuclear protein 1"
}